{
  "gene_name": "Transmembrane protease serine 9",
  "gene_symbol": "TMPRSS9",
  "term_label": "serine-type peptidase activity",
  "term_id": "GO:0008236",
  "gene": "UniProtKB:Q7Z410"
}